P2Y8 nucleotide receptor binding [GO:0031817] (molecular function) Also known as: P2Y8 nucleotide receptor ligand Sources: GOC:mah, GOC:nln Relationships: is a type of G protein-coupled nucleotide receptor binding [GO:0031811] Definition: Binding to a P2Y8 nucleotide receptor.